DNA/RNA hybrid binding [GO:0071667] (molecular function) Relationships: is a type of nucleic acid binding [GO:0003676] Also known as: RNA/DNA hybrid binding Definition: Binding to a RNA/DNA hybrid. Sources: GOC:ecd Subtypes: DNA/RNA hybrid annealing activity [GO:0097098]